{
  "gene": "UniProtKB:Q9H2F5",
  "gene_symbol": "EPC1",
  "term_label": "protein-macromolecule adaptor activity",
  "term_id": "GO:0030674",
  "gene_name": "Enhancer of polycomb homolog 1"
}